circadian regulation of heart rate by the suprachiasmatic nucleus [GO:0003055] (biological process) Sources: GOC:mtg_cardio, GOC:rl Relationships: is a type of circadian regulation of heart rate [GO:0003053] Also known as: SCN regulation of heart rate, master pacemaker clock regulation of heart rate, circadian regulation of heart contraction rate by the suprachiasmatic nucleus Definition: The process in which the suprachiasmatic nucleus modulates heart rate at different values with a regularity of approximately 24 hours.